{
  "term_id": "UNKNOWN:0003",
  "gene_symbol": "ARHGEF35",
  "gene_name": "Rho guanine nucleotide exchange factor 35",
  "term_label": "Unknown cellular component",
  "gene": "UniProtKB:A5YM69"
}